{
  "gene_symbol": "MCHR1",
  "gene": "UniProtKB:Q99705",
  "term_id": "GO:0043005",
  "term_label": "neuron projection",
  "gene_name": "Melanin-concentrating hormone receptor 1"
}